replisome [GO:0030894] (cellular component) Definition: A multi-component enzymatic machine at the replication fork which mediates DNA replication. Includes DNA primase, one or more DNA polymerases, DNA helicases, and other proteins. Sources: GOC:mah, GOC:vw Also known as: DNA synthesome complex, RC complex, replication-competent complex Relationships: is_a GO:0032993; BFO_0000050 replication fork [GO:0005657]; BFO_0000051 DNA helicase complex [GO:0033202]; has part DNA polymerase complex [GO:0042575] Subtypes: cytoplasmic replisome [GO:0043600], GO:0043601